{
  "term_label": "mitochondrial inner membrane",
  "gene": "UniProtKB:O75306",
  "term_id": "GO:0005743",
  "gene_name": "NADH dehydrogenase [ubiquinone] iron-sulfur protein 2, mitochondrial",
  "gene_symbol": "NDUFS2"
}